{
  "gene_name": "Glutamate receptor ionotropic, NMDA 2A",
  "gene": "UniProtKB:Q12879",
  "term_label": "NMDA selective glutamate receptor complex",
  "term_id": "GO:0017146",
  "gene_symbol": "GRIN2A"
}